{
  "gene": "UniProtKB:Q6H9L7",
  "term_id": "UNKNOWN:0001",
  "gene_symbol": "ISM2",
  "gene_name": "Isthmin-2",
  "term_label": "Unknown molecular function"
}